{
  "gene": "UniProtKB:O95816",
  "gene_symbol": "BAG2",
  "term_id": "GO:0000774",
  "gene_name": "BAG family molecular chaperone regulator 2",
  "term_label": "adenyl-nucleotide exchange factor activity"
}